{
  "term_label": "sarcolemma",
  "gene_name": "Blood vessel epicardial substance",
  "gene": "UniProtKB:Q8NE79",
  "gene_symbol": "BVES",
  "term_id": "GO:0042383"
}